{
  "term_label": "heterotrimeric G-protein complex",
  "gene_symbol": "GNGT2",
  "gene": "UniProtKB:O14610",
  "term_id": "GO:0005834",
  "gene_name": "Guanine nucleotide-binding protein G(I)_G(S)_G(O) subunit gamma-T2"
}